{
  "gene": "UniProtKB:Q5SY68",
  "term_label": "calcium ion binding",
  "gene_symbol": "S100A7L2",
  "term_id": "GO:0005509",
  "gene_name": "Protein S100-A7-like 2"
}